nucleoside phosphate catabolic process [GO:1901292] (BP) Sources: GOC:TermGenie Relationships: is a type of nucleoside phosphate metabolic process [GO:0006753]; is a type of nucleobase-containing compound catabolic process [GO:0034655]; is a type of GO:0046434 Definition: The chemical reactions and pathways resulting in the breakdown of a nucleoside phosphate. Also known as: nucleoside phosphate breakdown, nucleoside phosphate catabolism, nucleoside phosphate degradation Subtypes: nucleoside monophosphate catabolic process [GO:0009125], nucleoside diphosphate catabolic process [GO:0009134], GO:0009143, nucleotide catabolic process [GO:0009166], coenzyme A catabolic process [GO:0015938], nucleoside bisphosphate catabolic process [GO:0033869], fatty-acyl-CoA catabolic process [GO:0036115], acetyl-CoA catabolic process [GO:0046356], GO:1901289, benzoyl-CoA catabolic process [GO:1901788], 2-hydroxybenzoyl-CoA catabolic process [GO:1901886], malonyl-CoA catabolic process [GO:2001294]